{
  "term_id": "GO:0005759",
  "term_label": "mitochondrial matrix",
  "gene_symbol": "CCNB1",
  "gene_name": "G2_mitotic-specific cyclin-B1",
  "gene": "UniProtKB:P14635"
}